{
  "term_id": "GO:0004473",
  "term_label": "malate dehydrogenase (decarboxylating) (NADP+) activity",
  "gene_symbol": "ME2",
  "gene": "UniProtKB:P23368",
  "gene_name": "NAD-dependent malic enzyme, mitochondrial"
}